{
  "term_id": "GO:0005737",
  "term_label": "cytoplasm",
  "gene_symbol": "TNPO1",
  "gene_name": "Transportin-1",
  "gene": "UniProtKB:Q92973"
}